{
  "term_id": "GO:0048471",
  "term_label": "perinuclear region of cytoplasm",
  "gene_symbol": "CAV2",
  "gene": "UniProtKB:P51636",
  "gene_name": "Caveolin-2"
}